ribosomal protein import into nucleus [GO:0006610] (biological process) References: PMID:11809816 Sources: GOC:ai Definition: The directed movement of a ribosomal protein from the cytoplasm into the nucleus, across the nuclear membrane. At least some ribosomal proteins, including rpl12, uses the importin 11 pathway as a major route into the nucleus. Relationships: is a type of protein import into nucleus [GO:0006606] Note: Ribosomal protein rpl12 uses a different import pathway, which is why it has a separate GO term. Also known as: ribosomal protein import into cell nucleus, ribosomal protein transport from cytoplasm to nucleus, ribosomal protein-nucleus import